{
  "gene_symbol": "NPPC",
  "gene": "UniProtKB:P23582",
  "gene_name": "C-type natriuretic peptide",
  "term_label": "receptor guanylyl cyclase signaling pathway",
  "term_id": "GO:0007168"
}